purine nucleotide uniporter activity [GO:0160042] (molecular function) Relationships: is a type of purine nucleotide transmembrane transporter activity [GO:0015216]; is_a membrane potential driven uniporter activity [GO:0022810] References: PMID:18375752, PMID:27477609 Definition: Catalysis of the active transport of purine nucleotides across a membrane by a mechanism involving conformational change, where energy for active transport is derived from membrane potential if the solute is charged.